{
  "term_id": "UNKNOWN:0003",
  "gene": "UniProtKB:P17676",
  "gene_name": "CCAAT_enhancer-binding protein beta",
  "term_label": "Unknown cellular component",
  "gene_symbol": "CEBPB"
}